intracellular sodium ion homeostasis [GO:0006883] (BP) Sources: GOC:ai, GOC:mah Also known as: cellular sodium ion homeostasis Relationships: is a type of intracellular monoatomic cation homeostasis [GO:0030003]; is a type of GO:0055078 Definition: A homeostatic process involved in the maintenance of a steady state level of sodium ions within a cell.